{
  "gene": "UniProtKB:Q92581",
  "gene_symbol": "SLC9A6",
  "term_label": "potassium:proton antiporter activity",
  "gene_name": "Sodium_hydrogen exchanger 6",
  "term_id": "GO:0015386"
}